{
  "gene": "UniProtKB:P05937",
  "gene_name": "Calbindin",
  "gene_symbol": "CALB1",
  "term_label": "terminal bouton",
  "term_id": "GO:0043195"
}